{
  "term_id": "UNKNOWN:0003",
  "gene": "UniProtKB:Q5T7P2",
  "gene_name": "Late cornified envelope protein 1A",
  "gene_symbol": "LCE1A",
  "term_label": "Unknown cellular component"
}